{
  "term_label": "Unknown cellular component",
  "gene_name": "Putative uncharacterized protein encoded by LINC00869",
  "gene_symbol": "LINC00869",
  "gene": "UniProtKB:P0C866",
  "term_id": "UNKNOWN:0003"
}